{
  "gene_name": "Follistatin",
  "gene_symbol": "FST",
  "gene": "UniProtKB:P19883",
  "term_label": "activin binding",
  "term_id": "GO:0048185"
}